fatty acid alpha-dioxygenase activity [GO:0102672] (molecular function) Definition: Catalysis of the reaction: a 1,2-saturated fatty acid + O2 = a (2R)-2-hydroperoxy fatty acid. Sources: RHEA:63508 Also known as: fatty acid alpha-oxygenase activity Relationships: is a type of oxidoreductase activity, acting on single donors with incorporation of molecular oxygen, incorporation of two atoms of oxygen [GO:0016702]